{
  "gene_name": "Cilia- and flagella-associated protein 46",
  "term_label": "Unknown cellular component",
  "term_id": "UNKNOWN:0003",
  "gene_symbol": "CFAP46",
  "gene": "UniProtKB:Q8IYW2"
}